establishment of localization in cell [GO:0051649] (biological process) Subtypes: serotonin secretion by mast cell [GO:0002552], histamine secretion by mast cell [GO:0002553], serotonin secretion by platelet [GO:0002554], histamine secretion by platelet [GO:0002555], serotonin secretion by basophil [GO:0002556], histamine secretion by basophil [GO:0002557], platelet degranulation [GO:0002576], neurotransmitter secretion [GO:0007269], synaptic vesicle exocytosis [GO:0016079], iron import into cell [GO:0033212], insulin secretion involved in cellular response to glucose stimulus [GO:0035773], synaptic vesicle recycling [GO:0036465], GO:0043299, establishment of pole plasm mRNA localization [GO:0046595], GO:0046907, establishment of spindle localization [GO:0051293], GO:0051650, establishment of centrosome localization [GO:0051660], establishment of plastid localization [GO:0051667], establishment of Golgi localization [GO:0051683], establishment of ER localization [GO:0051686], substrate localization to autophagosome [GO:0061753], GO:0070560, establishment of protein localization to mitochondrial membrane [GO:0090151], synaptic vesicle lumen acidification [GO:0097401], neurotransmitter loading into synaptic vesicle [GO:0098700], neurotransmitter reuptake [GO:0098810], somato-dendritic dopamine secretion [GO:0099123], axonal dopamine secretion [GO:0099124], GO:0099504, release of sequestered calcium ion into presynaptic cytosol [GO:0099585], release of sequestered calcium ion into postsynaptic cytosol [GO:0099586], GO:0099606, postsynaptic neurotransmitter receptor cycle [GO:0099630], presynaptic endocytosis [GO:0140238], postsynaptic endocytosis [GO:0140239], GO:1905741, GO:1905743 Relationships: is a type of establishment of localization [GO:0051234]; is part of cellular localization [GO:0051641] Also known as: establishment of localisation in cell, establishment of intracellular localization, establishment of localization within cell, positioning within cell, establishment of cellular localization Definition: Any process, occurring in a cell, that localizes a substance or cellular component. This may occur via movement, tethering or selective degradation. Sources: GOC:ai, GOC:dos, GOC:dph, GOC:tb